{
  "gene_symbol": "PAGE4",
  "gene_name": "P antigen family member 4",
  "gene": "UniProtKB:O60829",
  "term_id": "UNKNOWN:0001",
  "term_label": "Unknown molecular function"
}